{
  "gene": "UniProtKB:Q15555",
  "gene_name": "Microtubule-associated protein RP_EB family member 2",
  "term_label": "protein localization to microtubule",
  "term_id": "GO:0035372",
  "gene_symbol": "MAPRE2"
}